{
  "gene": "UniProtKB:I0J062",
  "term_label": "Unknown molecular function",
  "term_id": "UNKNOWN:0001",
  "gene_name": "Proapoptotic nucleolar protein 1",
  "gene_symbol": "PANO1"
}